racemase and epimerase activity, acting on hydroxy acids and derivatives [GO:0016856] (molecular function) Subtypes: 3-hydroxybutyryl-CoA epimerase activity [GO:0008692], carnitine racemase activity [GO:0008809], mandelate racemase activity [GO:0018838], acetoin racemase activity [GO:0047604], isocitrate epimerase activity [GO:0047755], lactate racemase activity [GO:0050043], tartrate epimerase activity [GO:0050320] Relationships: is a type of racemase and epimerase activity [GO:0016854] Definition: Catalysis of a reaction that alters the configuration of one or more chiral centers in a hydroxy acid molecule. Sources: GOC:mah